{
  "gene_symbol": "RAB11FIP1",
  "gene_name": "Rab11 family-interacting protein 1",
  "gene": "UniProtKB:Q6WKZ4",
  "term_label": "Unknown cellular component",
  "term_id": "UNKNOWN:0003"
}